positive regulation of toll-like receptor 21 signaling pathway [GO:2000445] (biological process) Definition: Any process that activates or increases the frequency, rate or extent of toll-like receptor 21 signaling pathway. Sources: GOC:obol Also known as: positive regulation of TLR21 signaling pathway, positive regulation of toll-like receptor 21 signalling pathway Relationships: is a type of positive regulation of toll-like receptor signaling pathway [GO:0034123]; is a type of regulation of toll-like receptor 21 signaling pathway [GO:2000443]; positively regulates toll-like receptor 21 signaling pathway [GO:0035682]